{
  "term_id": "UNKNOWN:0001",
  "term_label": "Unknown molecular function",
  "gene_symbol": "DNAJC1",
  "gene": "UniProtKB:Q96KC8",
  "gene_name": "DnaJ homolog subfamily C member 1"
}